polyphenic determination, influence by genetic factors [GO:0048652] (biological process) Definition: The process in which individuals that have the potential to develop any of several possible distinct developmental paths have their individual developmental fates determined in response to genetic cues. Subtypes: caste determination, influence by genetic factors [GO:0048649] Sources: GOC:jid Relationships: is a type of polyphenic determination [GO:0048647]